{
  "term_label": "Unknown cellular component",
  "gene_symbol": "TMEM252",
  "term_id": "UNKNOWN:0003",
  "gene": "UniProtKB:Q8N6L7",
  "gene_name": "Transmembrane protein 252"
}